{
  "gene_symbol": "C18orf63",
  "term_label": "Unknown biological process",
  "gene_name": "Uncharacterized protein C18orf63",
  "term_id": "UNKNOWN:0002",
  "gene": "UniProtKB:Q68DL7"
}